{
  "gene_name": "Calcium_calmodulin-dependent protein kinase type II subunit gamma",
  "term_id": "GO:0014069",
  "gene_symbol": "CAMK2G",
  "gene": "UniProtKB:Q13555",
  "term_label": "postsynaptic density"
}